cellular response to lectin [GO:1990858] (biological process) References: PMID:25996210, PMID:26306444 Relationships: is a type of GO:1990840 Note: This term refers to endogenous (evolved) responses to lectins (endogenous or exogenous), it does not cover the events that happen due to lectin toxicity. Subtypes: GO:0002223 Definition: Any process that results in a change in state or activity of a cell (in terms of movement, secretion, enzyme production, gene expression, etc.) as a result of a lectin stimulus. A lectin is a carbohydrate-binding protein, highly specific for binding sugar moieties.